{
  "gene_symbol": "ZNF799",
  "term_id": "GO:0006357",
  "gene_name": "Zinc finger protein 799",
  "term_label": "regulation of transcription by RNA polymerase II",
  "gene": "UniProtKB:Q96GE5"
}